ADP-dependent NAD(P)H-hydrate dehydratase activity [GO:0052855] (molecular function) References: PMID:21994945 Sources: EC:4.2.1.136 Definition: Catalysis of the reaction: (6S)-6beta-hydroxy-1,4,5,6-tetrahydronicotinamide adenine dinucleotide + ADP = AMP + H+ + NAD(P)H + phosphate. Relationships: is a type of hydro-lyase activity [GO:0016836] Also known as: ADP-dependent H(4)NAD(P)OH dehydratase activity, ADP-dependent H4NAD(P)OH dehydratase activity, (6S)-beta-6-hydroxy-1,4,5,6-tetrahydronicotinamide-adenine-dinucleotide hydro-lyase (ADP-hydrolysing), (6S)-beta-6-hydroxy-1,4,5,6-tetrahydronicotinamide-adenine-dinucleotide hydro-lyase(ADP-hydrolysing; NADH-forming)